serine-type aminopeptidase activity [GO:0070009] (molecular function) Relationships: is a type of aminopeptidase activity [GO:0004177]; is a type of serine-type exopeptidase activity [GO:0070008] Definition: Catalysis of the hydrolysis of a single N-terminal amino acid residue from a polypeptide chain by a catalytic mechanism that involves a catalytic triad consisting of a serine nucleophile that is activated by a proton relay involving an acidic residue (e.g. aspartate or glutamate) and a basic residue (usually histidine). Sources: https://www.ebi.ac.uk/merops/about/glossary.shtml#AMINOPEPTIDASE, https://www.ebi.ac.uk/merops/about/glossary.shtml#CATTYPE